{
  "term_label": "adherens junction",
  "gene_name": "PDZ and LIM domain protein 3",
  "gene": "UniProtKB:Q53GG5",
  "term_id": "GO:0005912",
  "gene_symbol": "PDLIM3"
}